{
  "gene": "UniProtKB:Q9NR23",
  "gene_symbol": "GDF3",
  "gene_name": "Growth_differentiation factor 3",
  "term_id": "GO:0005125",
  "term_label": "cytokine activity"
}